carbohydrate derivative biosynthetic process [GO:1901137] (biological process) Subtypes: GO:0006023, GO:0006488, GO:0009101, lipopolysaccharide biosynthetic process [GO:0009103], nucleotide-sugar biosynthetic process [GO:0009226], colanic acid biosynthetic process [GO:0009242], enterobacterial common antigen biosynthetic process [GO:0009246], glycolipid biosynthetic process [GO:0009247], GO:0009248, deoxyribonucleotide biosynthetic process [GO:0009263], amylopectin biosynthetic process [GO:0010021], Lewis a epitope biosynthetic process [GO:0010493], teichoic acid biosynthetic process [GO:0019350], vancomycin biosynthetic process [GO:0033072], glyceraldehyde-3-phosphate biosynthetic process [GO:0046166], glycerol-3-phosphate biosynthetic process [GO:0046167], GO:0046349, deoxyribose phosphate biosynthetic process [GO:0046385], ribose phosphate biosynthetic process [GO:0046390], Lewis x epitope biosynthetic process [GO:0106402], GO:1901159, lipooligosaccharide biosynthetic process [GO:1901271], cyclic 2,3-bisphospho-D-glycerate biosynthetic process [GO:1901369], glycosyl compound biosynthetic process [GO:1901659], D-glycero-D-manno-heptose 7-phosphate biosynthetic process [GO:2001061], coenzyme gamma-F420-2 biosynthetic process [GO:2001121], lysobisphosphatidic acid biosynthetic process [GO:2001312] Definition: The chemical reactions and pathways resulting in the formation of carbohydrate derivative. Relationships: is a type of GO:0009058; is a type of carbohydrate derivative metabolic process [GO:1901135] Sources: GOC:TermGenie Also known as: carbohydrate derivative anabolism, carbohydrate derivative biosynthesis, carbohydrate derivative formation, carbohydrate derivative synthesis